{
  "gene_symbol": "RANGAP1",
  "gene_name": "Ran GTPase-activating protein 1",
  "term_label": "cytosol",
  "term_id": "GO:0005829",
  "gene": "UniProtKB:P46060"
}